{
  "gene_symbol": "POU4F2",
  "term_label": "regulation of transcription by RNA polymerase II",
  "gene": "UniProtKB:Q12837",
  "term_id": "GO:0006357",
  "gene_name": "POU domain, class 4, transcription factor 2"
}